{
  "gene_symbol": "C6orf120",
  "gene": "UniProtKB:Q7Z4R8",
  "gene_name": "UPF0669 protein C6orf120",
  "term_id": "UNKNOWN:0002",
  "term_label": "Unknown biological process"
}